{
  "term_id": "GO:0000014",
  "gene_symbol": "SETMAR",
  "gene_name": "Histone-lysine N-methyltransferase SETMAR",
  "gene": "UniProtKB:Q53H47",
  "term_label": "single-stranded DNA endodeoxyribonuclease activity"
}